cellular response to vitamin B6 [GO:0071304] (BP) Definition: Any process that results in a change in state or activity of a cell (in terms of movement, secretion, enzyme production, gene expression, etc.) as a result of a vitamin B6 stimulus. Vitamin B6 encompasses pyridoxal, pyridoxamine and pyridoxine and the active form, pyridoxal phosphate. Relationships: is a type of response to vitamin B6 [GO:0034516]; is_a cellular response to vitamin [GO:0071295]; is_a cellular response to nitrogen compound [GO:1901699]; is a type of cellular response to oxygen-containing compound [GO:1901701] Sources: GOC:mah